decylhomocitrate synthase activity [GO:0050458] (molecular function) Relationships: is a type of GO:0046912 Definition: Catalysis of the reaction: 2-oxoglutarate + H2O + lauroyl-CoA = (3S,4S)-3-hydroxytetradecane-1,3,4-tricarboxylate + CoA + H+. Sources: RHEA:10364 Also known as: 2-decylhomocitrate synthase activity, 3-hydroxytetradecane-1,3,4-tricarboxylate 2-oxoglutarate-lyase (CoA- acylating) activity, 3-hydroxytetradecane-1,3,4-tricarboxylate 2-oxoglutarate-lyase (CoA-acylating), dodecanoyl-CoA:2-oxoglutarate C-dodecanoyltransferase (thioester-hydrolysing, 1-carboxyundecyl-forming)